{
  "gene": "UniProtKB:A6NFE2",
  "term_label": "Unknown cellular component",
  "gene_name": "Single-pass membrane and coiled-coil domain-containing protein 2",
  "gene_symbol": "SMCO2",
  "term_id": "UNKNOWN:0003"
}